{
  "term_id": "GO:0043564",
  "term_label": "Ku70:Ku80 complex",
  "gene_symbol": "XRCC6",
  "gene_name": "X-ray repair cross-complementing protein 6",
  "gene": "UniProtKB:P12956"
}